protein localization to cell cortex of cell tip [GO:1990896] (biological process) Definition: A process in which a protein is transported to, or maintained in, the cell cortex of the cell tip. Relationships: is a type of protein localization to cell cortex [GO:0072697]; is a type of protein localization to cell tip [GO:1990151] Regulation: regulated by regulation of protein localization to cell cortex of cell tip [GO:1990895] Subtypes: microtubule polymerization based protein transport to cell tip cortex [GO:0099110] References: PMID:26150232